{
  "gene_symbol": "RNF144B",
  "term_id": "GO:0031966",
  "gene": "UniProtKB:Q7Z419",
  "term_label": "mitochondrial membrane",
  "gene_name": "E3 ubiquitin-protein ligase RNF144B"
}